{
  "term_label": "apical plasma membrane",
  "gene_name": "High affinity copper uptake protein 1",
  "term_id": "GO:0016324",
  "gene": "UniProtKB:O15431",
  "gene_symbol": "SLC31A1"
}